{
  "gene_symbol": "ARMC5",
  "gene": "UniProtKB:Q96C12",
  "term_id": "UNKNOWN:0001",
  "term_label": "Unknown molecular function",
  "gene_name": "Armadillo repeat-containing protein 5"
}